{
  "gene": "UniProtKB:Q9P0T7",
  "term_id": "UNKNOWN:0001",
  "term_label": "Unknown molecular function",
  "gene_symbol": "TMEM9",
  "gene_name": "Proton-transporting V-type ATPase complex assembly regulator TMEM9"
}